{
  "gene_name": "Zinc finger and SCAN domain-containing protein 9",
  "gene": "UniProtKB:O15535",
  "term_label": "RNA polymerase II cis-regulatory region sequence-specific DNA binding",
  "gene_symbol": "ZSCAN9",
  "term_id": "GO:0000978"
}